{
  "term_id": "GO:0010508",
  "term_label": "positive regulation of autophagy",
  "gene_symbol": "PRKAA2",
  "gene_name": "5'-AMP-activated protein kinase catalytic subunit alpha-2",
  "gene": "UniProtKB:P54646"
}